{
  "gene_symbol": "SS18L1",
  "gene_name": "Calcium-responsive transactivator",
  "gene": "UniProtKB:O75177",
  "term_id": "GO:0050775",
  "term_label": "positive regulation of dendrite morphogenesis"
}